creation date [oboInOwl#creation:date]